{
  "gene": "UniProtKB:Q7L523",
  "term_id": "GO:1990131",
  "gene_symbol": "RRAGA",
  "gene_name": "Ras-related GTP-binding protein A",
  "term_label": "Gtr1-Gtr2 GTPase complex"
}